{
  "term_label": "protein phosphatase 4 complex",
  "term_id": "GO:0030289",
  "gene": "UniProtKB:Q6IN85",
  "gene_symbol": "PPP4R3A",
  "gene_name": "Serine_threonine-protein phosphatase 4 regulatory subunit 3A"
}